meiotic cell cycle phase transition [GO:0044771] (biological process) Sources: GOC:mtg_cell_cycle Relationships: is a type of cell cycle phase transition [GO:0044770]; is a type of meiotic cell cycle process [GO:1903046] Subtypes: G2/MI transition of meiotic cell cycle [GO:0008315], metaphase/anaphase transition of meiotic cell cycle [GO:0044785], GO:1990946, GO:1990947 Definition: The cell cycle process by which a cell commits to entering the next meiotic cell cycle phase. Regulation: RO_0002211 by regulation of meiotic cell cycle phase transition [GO:1901993]; negatively regulated by negative regulation of meiotic cell cycle phase transition [GO:1901994]; positively regulated by positive regulation of meiotic cell cycle phase transition [GO:1901995] Also known as: cell cycle transition